{
  "term_label": "multimeric ribonuclease P complex",
  "gene_name": "Ribonuclease P protein subunit p14",
  "gene": "UniProtKB:O95059",
  "term_id": "GO:0030681",
  "gene_symbol": "RPP14"
}